malonic acid transmembrane transport [GO:1901553] (biological process) Note: Note that this term is not intended for use in annotating lateral movement within membranes. Definition: The directed movement of malonic acid across a membrane. Subtypes: malonic acid import across plasma membrane [GO:0098715], mitochondrial malonate(1-) transmembrane transport [GO:1990558] Also known as: malonic acid membrane transport Relationships: is a type of malonic acid transport [GO:1900752]; is a type of carboxylic acid transmembrane transport [GO:1905039] Sources: GOC:TermGenie, GOC:al